negative regulation of endocytosis [GO:0045806] (biological process) Subtypes: negative regulation of receptor-mediated endocytosis [GO:0048261], negative regulation of pinocytosis [GO:0048550], negative regulation of phagocytosis [GO:0050765], negative regulation of synaptic vesicle endocytosis [GO:1900243], negative regulation of ubiquitin-dependent endocytosis [GO:2000396], negative regulation of caveolin-mediated endocytosis [GO:2001287] Sources: GOC:go_curators Definition: Any process that stops, prevents, or reduces the frequency, rate or extent of endocytosis. Also known as: down regulation of endocytosis, down-regulation of endocytosis, downregulation of endocytosis, inhibition of endocytosis Relationships: is a type of GO:0030100; is a type of GO:0051051; is a type of negative regulation of cellular component organization [GO:0051129]; negatively regulates GO:0006897